{
  "gene_symbol": "B3GNT6",
  "term_label": "galactosyltransferase activity",
  "term_id": "GO:0008378",
  "gene": "UniProtKB:Q6ZMB0",
  "gene_name": "Acetylgalactosaminyl-O-glycosyl-glycoprotein beta-1,3-N-acetylglucosaminyltransferase"
}